{
  "gene": "UniProtKB:Q96PB7",
  "term_id": "GO:0007165",
  "gene_symbol": "OLFM3",
  "gene_name": "Noelin-3",
  "term_label": "signal transduction"
}